{
  "gene": "UniProtKB:O60675",
  "term_id": "GO:0005634",
  "gene_name": "Transcription factor MafK",
  "gene_symbol": "MAFK",
  "term_label": "nucleus"
}